iodide transport [GO:0015705] (biological process) Subtypes: GO:1904200 Sources: GOC:krc Definition: The directed movement of iodide into, out of or within a cell, or between cells, by means of some agent such as a transporter or pore. Relationships: is a type of monoatomic anion transport [GO:0006820]; is a type of GO:0015698 Regulation: regulated by GO:1904201; negatively regulated by negative regulation of iodide transport [GO:1904202]; positively regulated by positive regulation of iodide transport [GO:1904203]